{
  "gene_symbol": "DEFA6",
  "term_id": "GO:0140911",
  "gene": "UniProtKB:Q01524",
  "gene_name": "Defensin-6",
  "term_label": "pore-forming activity"
}